{
  "term_label": "syntaxin binding",
  "term_id": "GO:0019905",
  "gene_name": "Synaptosomal-associated protein 29",
  "gene": "UniProtKB:O95721",
  "gene_symbol": "SNAP29"
}